{
  "gene": "UniProtKB:Q9P2P5",
  "gene_name": "E3 ubiquitin-protein ligase HECW2",
  "term_label": "ubiquitin-dependent protein catabolic process",
  "term_id": "GO:0006511",
  "gene_symbol": "HECW2"
}